{
  "gene_name": "GPI ethanolamine phosphate transferase 2",
  "term_id": "GO:0006506",
  "gene": "UniProtKB:Q5H8A4",
  "gene_symbol": "PIGG",
  "term_label": "GPI anchor biosynthetic process"
}